negative regulation of focal adhesion disassembly [GO:0120184] (biological process) Definition: Any process that stops, prevents, or reduces the frequency, rate or extent of a focal adhesion into its constituent components. Relationships: is a type of GO:0120182; is a type of negative regulation of cell-substrate junction organization [GO:0150118]; negatively regulates focal adhesion disassembly [GO:0120181] References: PMID:25490267